{
  "gene_symbol": "C8orf58",
  "term_label": "Unknown cellular component",
  "gene": "UniProtKB:Q8NAV2",
  "gene_name": "Uncharacterized protein C8orf58",
  "term_id": "UNKNOWN:0003"
}